{
  "gene_name": "GSK-3-binding protein FRAT2",
  "term_label": "Unknown biological process",
  "gene": "UniProtKB:O75474",
  "gene_symbol": "FRAT2",
  "term_id": "UNKNOWN:0002"
}